cell recognition [GO:0008037] (biological process) Subtypes: phagocytosis, recognition [GO:0006910], GO:0008038, GO:0009988, cell-matrix recognition [GO:0009989], GO:0048544 Definition: The process in which a cell in an organism interprets its surroundings. Also known as: recognition of surroundings by cell Relationships: is a type of cellular process [GO:0009987] Sources: GOC:go_curators